{
  "gene_symbol": "TMEM94",
  "gene": "UniProtKB:Q12767",
  "term_id": "GO:0005789",
  "term_label": "endoplasmic reticulum membrane",
  "gene_name": "Transmembrane protein 94"
}